{
  "term_id": "GO:0007155",
  "gene_name": "Protocadherin beta-15",
  "gene": "UniProtKB:Q9Y5E8",
  "term_label": "cell adhesion",
  "gene_symbol": "PCDHB15"
}